substance P catabolic process [GO:0010814] (biological process) Relationships: is a type of neuropeptide catabolic process [GO:0010813]; is a type of amide metabolic process [GO:0043603] Sources: GOC:BHF, GOC:rl Definition: The chemical reactions and pathways resulting in the breakdown of the neuropeptide substance P.